{
  "gene": "UniProtKB:Q9Y6P5",
  "term_id": "GO:0016684",
  "gene_symbol": "SESN1",
  "term_label": "oxidoreductase activity, acting on peroxide as acceptor",
  "gene_name": "Sestrin-1"
}